{
  "gene_symbol": "UVSSA",
  "gene_name": "UV-stimulated scaffold protein A",
  "term_label": "response to UV",
  "term_id": "GO:0009411",
  "gene": "UniProtKB:Q2YD98"
}